petal morphogenesis [GO:0048446] (biological process) Sources: GOC:go_curators Relationships: is a type of floral organ morphogenesis [GO:0048444]; is part of petal development [GO:0048441] Definition: The process in which the anatomical structures of the petal are generated and organized.